{
  "gene": "UniProtKB:Q9BTP7",
  "gene_name": "Fanconi anemia core complex-associated protein 24",
  "term_id": "GO:0043240",
  "term_label": "Fanconi anaemia nuclear complex",
  "gene_symbol": "FAAP24"
}